{
  "term_id": "UNKNOWN:0003",
  "term_label": "Unknown cellular component",
  "gene_symbol": "NOS1AP",
  "gene": "UniProtKB:O75052",
  "gene_name": "Carboxyl-terminal PDZ ligand of neuronal nitric oxide synthase protein"
}